{
  "gene": "UniProtKB:Q6PFW1",
  "gene_symbol": "PPIP5K1",
  "term_id": "GO:0005829",
  "gene_name": "Inositol hexakisphosphate and diphosphoinositol-pentakisphosphate kinase 1",
  "term_label": "cytosol"
}